ACA codon-amino acid adaptor activity [GO:0033439] (molecular function) Note: Note that in the standard genetic code, ACA codes for threonine. Definition: A triplet codon-amino acid adaptor activity that recognizes an ACA codon. Sources: GOC:mah Also known as: threonine tRNA Relationships: is a type of triplet codon-amino acid adaptor activity [GO:0030533]